positive regulation of Rac protein signal transduction [GO:0035022] (biological process) Sources: GOC:bf Relationships: is a type of GO:0035020; is a type of GO:0051057; positively regulates GO:0016601 Definition: Any process that activates or increases the frequency, rate or extent of Rac protein signal transduction. Also known as: up regulation of Rac protein signal transduction, up-regulation of Rac protein signal transduction, upregulation of Rac protein signal transduction, activation of Rac protein signal transduction, stimulation of Rac protein signal transduction